tRNA guanylyltransferase activity [GO:0008193] (molecular function) Definition: Catalysis of the posttranscriptional addition of a guanyl residue to the 5' end of a tRNA molecule; observed for His tRNAs. Relationships: is a type of RNA guanylyltransferase activity [GO:0008192]; is_a GO:0140101; is part of tRNA 5'-end processing [GO:0099116] References: PMID:1660461